positive regulation of granzyme B production [GO:0071663] (biological process) Definition: Any process that activates or increases the frequency, rate, or extent of production of granzyme B. Sources: GOC:mah Relationships: is a type of positive regulation of production of molecular mediator of immune response [GO:0002702]; is a type of regulation of granzyme B production [GO:0071661]; positively regulates granzyme B production [GO:0071613]